N-1-naphthylphthalamic acid binding [GO:0010013] (molecular function) Definition: Binding to N-1-naphthylphthalamic acid, an auxin transport inhibitor. Relationships: is_a GO:0033218; is a type of monocarboxylic acid binding [GO:0033293] Sources: GOC:sm